{
  "gene_name": "Dynamin-1",
  "term_id": "GO:0005737",
  "term_label": "cytoplasm",
  "gene_symbol": "DNM1",
  "gene": "UniProtKB:Q05193"
}